{
  "gene_name": "Protein-tyrosine kinase 2-beta",
  "gene_symbol": "PTK2B",
  "term_id": "GO:0004715",
  "gene": "UniProtKB:Q14289",
  "term_label": "non-membrane spanning protein tyrosine kinase activity"
}